positive regulation of IRE1-mediated unfolded protein response [GO:1903896] (biological process) Definition: Any process that activates or increases the frequency, rate or extent of the IRE1-mediated unfolded protein response. References: PMID:22013210 Sources: GOC:PARL, GOC:TermGenie, GOC:bf, GO_REF:0000058 Also known as: positive regulation of IRE1 branch of UPR, positive regulation of UPR signaling by IRE1 stress sensor, positive regulation of endoplasmic reticulum unfolded protein response; IRE1 signaling, up regulation of IRE1 branch of UPR, up regulation of IRE1-mediated unfolded protein response, up regulation of UPR signaling by IRE1 stress sensor, up regulation of endoplasmic reticulum unfolded protein response; IRE1 signaling, up-regulation of IRE1 branch of UPR, up-regulation of IRE1-mediated unfolded protein response, up-regulation of UPR signaling by IRE1 stress sensor, up-regulation of endoplasmic reticulum unfolded protein response; IRE1 signaling, upregulation of IRE1 branch of UPR, upregulation of IRE1-mediated unfolded protein response, upregulation of UPR signaling by IRE1 stress sensor, upregulation of endoplasmic reticulum unfolded protein response; IRE1 signaling, activation of IRE1 branch of UPR, activation of IRE1-mediated unfolded protein response, activation of IRE1alpha unfolded protein response, activation of IRE1p unfolded protein response, activation of UPR signaling by IRE1 stress sensor, activation of endoplasmic reticulum unfolded protein response; IRE1 signaling, positive regulation of IRE1alpha unfolded protein response, positive regulation of IRE1p unfolded protein response, up regulation of IRE1alpha unfolded protein response, up regulation of IRE1p unfolded protein response, up-regulation of IRE1alpha unfolded protein response, up-regulation of IRE1p unfolded protein response, upregulation of IRE1alpha unfolded protein response, upregulation of IRE1p unfolded protein response, activation of IRE1 signaling in response to endoplasmic reticulum stress, activation of inositol-requiring transmembrane kinase/endonuclease signal transduction, positive regulation of ERN1-mediated unfolded protein response, positive regulation of IRE1 signaling in response to endoplasmic reticulum stress, positive regulation of inositol-requiring transmembrane kinase/endonuclease signal transduction, up regulation of IRE1 signaling in response to endoplasmic reticulum stress, up regulation of inositol-requiring transmembrane kinase/endonuclease signal transduction, up-regulation of IRE1 signaling in response to endoplasmic reticulum stress, up-regulation of inositol-requiring transmembrane kinase/endonuclease signal transduction, upregulation of IRE1 signaling in response to endoplasmic reticulum stress, upregulation of inositol-requiring transmembrane kinase/endonuclease signal transduction Relationships: is a type of positive regulation of endoplasmic reticulum unfolded protein response [GO:1900103]; is a type of regulation of IRE1-mediated unfolded protein response [GO:1903894]; RO_0002213 IRE1-mediated unfolded protein response [GO:0036498]